branchiomotor neuron axon guidance in branchial arch mesenchyme [GO:0021789] (biological process) Relationships: is_a branchiomotor neuron axon guidance [GO:0021785] Subtypes: GO:0021790, chemoattraction of branchiomotor neuron axon in branchial arch mesenchyme [GO:0021791] References: PMID:14699587 Sources: GOC:cls, GOC:dgh, GOC:dph, GOC:jid, GO_REF:0000021 Definition: The process in which a branchiomotor neuron growth cone in the branchial arch mesenchyme is directed to a specific target site in the branchial arch mesenchyme. Branchiomotor neurons are located in the hindbrain and innervate branchial arch-derived muscles that control jaw movements, facial expression, the larynx, and the pharynx.